{
  "gene": "UniProtKB:Q9BX93",
  "gene_name": "Group XIIB secretory phospholipase A2-like protein",
  "term_id": "UNKNOWN:0001",
  "term_label": "Unknown molecular function",
  "gene_symbol": "PLA2G12B"
}